cellular response to thyrotropin-releasing hormone [GO:1905229] (biological process) Also known as: cellular response to protirelin, cellular response to TRH Relationships: is a type of GO:0071375; is a type of response to thyrotropin-releasing hormone [GO:1905225] References: PMID:21382270 Sources: GOC:TermGenie, GO_REF:0000071 Definition: Any process that results in a change in state or activity of a cell (in terms of movement, secretion, enzyme production, gene expression, etc.) as a result of a thyrotropin-releasing hormone (TRH) stimulus. TRH increases the secretion of thyroid-stimulating hormone by the anterior pituitary.